[hydroxymethylglutaryl-CoA reductase (NADPH)] kinase activity [GO:0047322] (molecular function) Relationships: is_a protein serine/threonine kinase activity [GO:0004674] Also known as: reductase kinase activity, 3-hydroxy-3-methylglutaryl coenzyme A reductase kinase activity, 3-hydroxy-3-methylglutaryl-CoA reductase kinase activity, AMPK, ATP:hydroxymethylglutaryl-CoA reductase (NADPH) phosphotransferase activity, HMG-CoA reductase kinase activity, STK29, beta-hydroxy-beta-methylglutaryl-CoA reductase kinase activity, hydroxymethylglutaryl coenzyme A reductase kinase (phosphorylating) activity, hydroxymethylglutaryl coenzyme A reductase kinase activity, hydroxymethylglutaryl-CoA reductase (NADPH) kinase activity, hydroxymethylglutaryl-CoA reductase (NADPH2) kinase activity, hydroxymethylglutaryl-CoA reductase kinase activity Definition: Catalysis of the reaction: [3-hydroxy-3-methylglutaryl-CoA reductase (NADPH)] + ATP = [3-hydroxy-3-methylglutaryl-CoA reductase (NADPH)] phosphate + ADP. Sources: EC:2.7.11.31